{
  "term_label": "ribosomal large subunit export from nucleus",
  "gene_symbol": "NMD3",
  "gene": "UniProtKB:Q96D46",
  "gene_name": "60S ribosomal export protein NMD3",
  "term_id": "GO:0000055"
}